{
  "gene_name": "Neuroplastin",
  "term_id": "GO:0007411",
  "term_label": "axon guidance",
  "gene": "UniProtKB:Q9Y639",
  "gene_symbol": "NPTN"
}